{
  "gene": "UniProtKB:Q13023",
  "gene_symbol": "AKAP6",
  "term_label": "regulation of membrane repolarization",
  "term_id": "GO:0060306",
  "gene_name": "A-kinase anchor protein 6"
}